{
  "gene": "UniProtKB:Q5BVD1",
  "gene_name": "TPA-induced transmembrane protein",
  "term_label": "Unknown biological process",
  "gene_symbol": "TTMP",
  "term_id": "UNKNOWN:0002"
}